{
  "gene": "UniProtKB:P02751",
  "gene_symbol": "FN1",
  "term_label": "cell-substrate junction assembly",
  "gene_name": "Fibronectin",
  "term_id": "GO:0007044"
}